{
  "term_label": "plasma membrane",
  "gene_name": "Low-density lipoprotein receptor",
  "gene": "UniProtKB:P01130",
  "term_id": "GO:0005886",
  "gene_symbol": "LDLR"
}